{
  "term_label": "Unknown biological process",
  "gene_name": "Coiled-coil domain-containing protein 157",
  "term_id": "UNKNOWN:0002",
  "gene_symbol": "CCDC157",
  "gene": "UniProtKB:Q569K6"
}